{
  "gene_symbol": "CD22",
  "gene": "UniProtKB:P20273",
  "term_label": "negative regulation of B cell receptor signaling pathway",
  "gene_name": "B-cell receptor CD22",
  "term_id": "GO:0050859"
}